negative regulation of neosartoricin biosynthetic process [GO:1902054] (biological process) Definition: Any process that stops, prevents or reduces the frequency, rate or extent of neosartoricin biosynthetic process. Relationships: is a type of negative regulation of polyketide biosynthetic process [GO:1900733]; is a type of GO:1902053; is a type of negative regulation of alcohol biosynthetic process [GO:1902931]; negatively regulates neosartoricin biosynthetic process [GO:1902050] References: PMID:23368997 Sources: GOC:TermGenie, GOC:di Also known as: down regulation of neosartoricin anabolism, down regulation of neosartoricin biosynthesis, down regulation of neosartoricin biosynthetic process, down regulation of neosartoricin formation, down regulation of neosartoricin synthesis, down-regulation of neosartoricin anabolism, down-regulation of neosartoricin biosynthesis, down-regulation of neosartoricin biosynthetic process, down-regulation of neosartoricin formation, down-regulation of neosartoricin synthesis, downregulation of neosartoricin anabolism, downregulation of neosartoricin biosynthesis, downregulation of neosartoricin biosynthetic process, downregulation of neosartoricin formation, downregulation of neosartoricin synthesis, inhibition of neosartoricin anabolism, inhibition of neosartoricin biosynthesis, inhibition of neosartoricin formation, inhibition of neosartoricin synthesis, negative regulation of neosartoricin anabolism, negative regulation of neosartoricin biosynthesis, negative regulation of neosartoricin formation, negative regulation of neosartoricin synthesis, inhibition of neosartoricin biosynthetic process